cell motility involved in cerebral cortex radial glia guided migration [GO:0021814] (BP) Definition: The movement of a cell along the process of a radial glial cell involved in cerebral cortex glial-mediated radial migration. Relationships: is a type of cell motility [GO:0048870]; is part of cerebral cortex radial glia-guided migration [GO:0021801] Also known as: cell locomotion involved in cerebral cortex glial-mediated radial migration, cell locomotion involved in cerebral cortex radial glia guided migration References: PMID:12626695 Sources: GOC:cls, GOC:dgh, GOC:dph, GOC:jid, GO_REF:0000021 Regulation: negatively regulated by negative regulation of cell motility involved in cerebral cortex radial glia guided migration [GO:0021822]